{
  "gene_name": "Cyclin-dependent kinase 11B",
  "term_id": "GO:0005634",
  "gene": "UniProtKB:P21127",
  "term_label": "nucleus",
  "gene_symbol": "CDK11B"
}